UFD1-NPL4 complex [GO:0036501] (cellular component) Relationships: is a type of protein-containing complex [GO:0032991]; BFO_0000050 cytoplasm [GO:0005737] Also known as: Npl4p-Ufd1p complex, UFD1L-NPLOC4 complex, Ufd1-Npl4 binary complex, Ufd1-Npl4 cofactor complex, Ufd1/Npl4 complex Definition: A dimeric protein complex that contains the co-factors for the ATPase VCP/p97 (Cdc48p in budding yeast). In mammals, this complex consists of UFD1L (UFD1) and NPLOC4 (NPL4). In budding yeast, the complex is a dimer of Ufd1p and Npl4p. References: PMID:10811609, PMID:17289586 Sources: GOC:PARL, GOC:bf